{
  "term_id": "UNKNOWN:0001",
  "gene_symbol": "OCIAD1",
  "gene": "UniProtKB:Q9NX40",
  "gene_name": "OCIA domain-containing protein 1",
  "term_label": "Unknown molecular function"
}